{
  "term_id": "GO:0006886",
  "gene_name": "Transmembrane emp24 domain-containing protein 10",
  "gene_symbol": "TMED10",
  "gene": "UniProtKB:P49755",
  "term_label": "intracellular protein transport"
}